protein-membrane adaptor activity [GO:0043495] (molecular function) Also known as: protein membrane adaptor, protein membrane adaptor activity, anchoring, protein membrane anchor Relationships: is a type of protein-macromolecule adaptor activity [GO:0030674] Definition: The binding activity of a molecule that brings together a protein or a protein complex with a membrane, either via membrane lipid binding or by interacting with a membrane protein, to establish or maintain the localization of the protein, protein complex or organelle. Sources: GOC:go_curators Subtypes: double strand break-nuclear membrane anchor activity [GO:0062241], cytoskeletal protein-membrane anchor activity [GO:0106006], spindle pole body-nuclear membrane anchor activity [GO:0106166], mitochondrion-plasma membrane adaptor activity [GO:0140443], GO:0140444, GO:0140449, telomere-nuclear envelope anchor activity [GO:0140473], GO:0140707, autophagosome-membrane adaptor activity [GO:0160183], peroxisome-mitochondrion membrane tether activity [GO:0160190], mitochondrion-mitochondrion outer membrane tether activity [GO:0160204], endoplasmic reticulum-plasma membrane adaptor activity [GO:0160214], endoplasmic reticulum-lipid droplet tether activity [GO:0170007], endoplasmic reticulum-organelle membrane tether activity [GO:0170009], protein-mitochondrial outer membrane tethering activity [GO:0180050], proteasome-nuclear membrane anchor activity [GO:1990919]